regulation of sclerotome development [GO:0061190] (biological process) Definition: Any process that modulates the rate, frequency, or extent of the progression of the sclerotome over time, from its initial formation to the mature structure. The sclerotome is the portion of the somite that will give rise to a vertebra. Sources: GOC:dph Relationships: is a type of regulation of developmental process [GO:0050793]; regulates sclerotome development [GO:0061056] Subtypes: GO:0061189